{
  "gene_name": "ICOS ligand",
  "term_label": "external side of plasma membrane",
  "gene_symbol": "ICOSLG",
  "term_id": "GO:0009897",
  "gene": "UniProtKB:O75144"
}